endoplasmic reticulum-autophagosome adaptor activity [GO:0140506] (molecular function) Relationships: is a type of autophagosome-membrane adaptor activity [GO:0160183]; is a type of endoplasmic reticulum-organelle membrane tether activity [GO:0170009] Also known as: ER- autophagosome anchor, autophagosome-ER anchor, autophagosome-endoplasmic reticulum anchor Definition: The binding activity of a molecule that brings together an ER membrane and an autophagosome during reticulophagy. References: PMID:32735772